{
  "gene_name": "Eukaryotic elongation factor 2 kinase",
  "term_id": "GO:0014069",
  "term_label": "postsynaptic density",
  "gene_symbol": "EEF2K",
  "gene": "UniProtKB:O00418"
}